protein sulfhydration [GO:0044524] (biological process) Definition: The modification of a protein amino acid by the addition of sulfur. References: PMID:19903941, PMID:22169477, PMID:8161529 Sources: GOC:jl, GOC:jsg Relationships: is a type of protein modification process [GO:0036211] Subtypes: peptidyl-cystine sulfhydration [GO:0044525]